{
  "gene": "UniProtKB:O94892",
  "term_label": "Unknown molecular function",
  "gene_name": "Zinc finger protein 432",
  "gene_symbol": "ZNF432",
  "term_id": "UNKNOWN:0001"
}